{
  "term_label": "3-hydroxyacyl-CoA dehydratase activity",
  "gene_symbol": "HACD2",
  "gene": "UniProtKB:Q6Y1H2",
  "term_id": "GO:0018812",
  "gene_name": "Very-long-chain (3R)-3-hydroxyacyl-CoA dehydratase 2"
}